positive regulation of leukocyte chemotaxis [GO:0002690] (BP) Sources: GOC:add Also known as: positive regulation of immune cell chemotaxis, positive regulation of leucocyte chemotaxis, up regulation of leukocyte chemotaxis, up-regulation of leukocyte chemotaxis, upregulation of leukocyte chemotaxis, activation of leukocyte chemotaxis, stimulation of leukocyte chemotaxis Subtypes: positive regulation of macrophage chemotaxis [GO:0010759], GO:0060754, positive regulation of granulocyte chemotaxis [GO:0071624], positive regulation of monocyte chemotaxis [GO:0090026], GO:0140131, positive regulation of dendritic cell chemotaxis [GO:2000510] Definition: Any process that activates or increases the frequency, rate, or extent of leukocyte chemotaxis. Relationships: is a type of positive regulation of leukocyte migration [GO:0002687]; is a type of GO:0002688; is a type of positive regulation of chemotaxis [GO:0050921]; positively regulates GO:0030595